{
  "term_id": "GO:0061668",
  "gene_symbol": "MTERF3",
  "gene": "UniProtKB:Q96E29",
  "term_label": "mitochondrial ribosome assembly",
  "gene_name": "Transcription termination factor 3, mitochondrial"
}